{
  "gene": "UniProtKB:Q9UQ49",
  "gene_symbol": "NEU3",
  "term_label": "ganglioside catabolic process",
  "term_id": "GO:0006689",
  "gene_name": "Sialidase-3"
}